{
  "gene": "UniProtKB:P06703",
  "term_id": "GO:0005634",
  "gene_name": "Protein S100-A6",
  "gene_symbol": "S100A6",
  "term_label": "nucleus"
}